{
  "gene_symbol": "AQP3",
  "gene": "UniProtKB:Q92482",
  "term_label": "glycerol transmembrane transport",
  "term_id": "GO:0015793",
  "gene_name": "Aquaporin-3"
}